{
  "gene_name": "Zinc finger protein 138",
  "term_label": "RNA polymerase II cis-regulatory region sequence-specific DNA binding",
  "gene": "UniProtKB:P52744",
  "gene_symbol": "ZNF138",
  "term_id": "GO:0000978"
}